{
  "gene_name": "Ribosomal protein eL42-like",
  "term_id": "GO:0003735",
  "gene": "UniProtKB:Q969Q0",
  "gene_symbol": "RPL36AL",
  "term_label": "structural constituent of ribosome"
}